{
  "term_id": "UNKNOWN:0003",
  "gene": "UniProtKB:Q8N446",
  "term_label": "Unknown cellular component",
  "gene_name": "Zinc finger protein 843",
  "gene_symbol": "ZNF843"
}